3-hydroxyphenylacetate catabolic process [GO:0019610] (biological process) Also known as: 3-hydroxyphenylacetate breakdown, 3-hydroxyphenylacetate catabolism, 3-hydroxyphenylacetate degradation Relationships: is a type of GO:0019336; is a type of xenobiotic catabolic process [GO:0042178]; is a type of monocarboxylic acid catabolic process [GO:0072329] References: PMID:6995433 Definition: The chemical reactions and pathways resulting in the breakdown of 3-hydroxyphenylacetate, 1,3-benzenediol monoacetate, also known as resorcinol monoacetate.